{
  "term_id": "GO:0005886",
  "gene_name": "Plexin-B2",
  "gene": "UniProtKB:O15031",
  "term_label": "plasma membrane",
  "gene_symbol": "PLXNB2"
}